positive regulation of chromatin binding [GO:0035563] (biological process) Relationships: is a type of positive regulation of binding [GO:0051099]; positively regulates GO:0003682 Definition: Any process that increases the frequency, rate or extent of chromatin binding. Chromatin binding is the selective interaction with chromatin, the network of fibers of DNA, protein, and sometimes RNA, that make up the chromosomes of the eukaryotic nucleus during interphase. References: PMID:20404130 Sources: GOC:bf